{
  "gene": "UniProtKB:Q5JTD7",
  "term_id": "UNKNOWN:0003",
  "gene_symbol": "LRRC73",
  "gene_name": "Leucine-rich repeat-containing protein 73",
  "term_label": "Unknown cellular component"
}